{
  "gene_name": "CD44 antigen",
  "gene_symbol": "CD44",
  "term_id": "GO:0004896",
  "term_label": "cytokine receptor activity",
  "gene": "UniProtKB:P16070"
}